{
  "term_label": "endocytic vesicle",
  "term_id": "GO:0030139",
  "gene_symbol": "EHD2",
  "gene_name": "EH domain-containing protein 2",
  "gene": "UniProtKB:Q9NZN4"
}